{
  "term_label": "single-stranded 3'-5' DNA helicase activity",
  "gene_symbol": "MCM6",
  "term_id": "GO:1990518",
  "gene_name": "DNA replication licensing factor MCM6",
  "gene": "UniProtKB:Q14566"
}